negative regulation of termination of RNA polymerase I transcription [GO:2000731] (biological process) Relationships: is a type of GO:0016479; is a type of negative regulation of termination of DNA-templated transcription [GO:0060567]; is a type of regulation of termination of RNA polymerase I transcription [GO:2000730]; negatively regulates GO:0006363 Sources: GOC:obol Also known as: negative regulation of RNA polymerase I transcription termination, negative regulation of transcription termination from Pol I promoter, negative regulation of transcription termination from RNA polymerase I promoter Definition: Any process that stops, prevents or reduces the frequency, rate or extent of termination of RNA polymerase I transcription.